{
  "gene_symbol": "SPTAN1",
  "term_id": "GO:0030864",
  "term_label": "cortical actin cytoskeleton",
  "gene_name": "Spectrin alpha chain, non-erythrocytic 1",
  "gene": "UniProtKB:Q13813"
}